glutamate-tRNA ligase activity [GO:0004818] (molecular function) Relationships: is a type of aminoacyl-tRNA ligase activity [GO:0004812] Sources: EC:6.1.1.17 Also known as: glutamyl-tRNA synthetase activity, L-glutamate:tRNAGlu ligase (AMP-forming) activity, glutamate-tRNA synthetase activity, glutamic acid translase activity, glutamyl-transfer RNA synthetase activity, glutamyl-transfer ribonucleate synthetase activity, glutamyl-transfer ribonucleic acid synthetase activity Definition: Catalysis of the reaction: ATP + L-glutamate + tRNA(Glu) = AMP + diphosphate + L-glutamyl-tRNA(Glu).